{
  "gene_symbol": "SPDYE5",
  "gene_name": "Speedy protein E5",
  "term_id": "GO:0019901",
  "gene": "UniProtKB:A6NIY4",
  "term_label": "protein kinase binding"
}